{
  "term_id": "GO:0005654",
  "gene_name": "Proteasome activator complex subunit 1",
  "gene": "UniProtKB:Q06323",
  "term_label": "nucleoplasm",
  "gene_symbol": "PSME1"
}